{
  "term_label": "response to exogenous dsRNA",
  "gene_name": "Interferon epsilon",
  "gene": "UniProtKB:Q86WN2",
  "term_id": "GO:0043330",
  "gene_symbol": "IFNE"
}